{
  "term_label": "DNA-binding transcription factor activity, RNA polymerase II-specific",
  "gene_symbol": "ZNF260",
  "gene_name": "Zinc finger protein 260",
  "gene": "UniProtKB:Q3ZCT1",
  "term_id": "GO:0000981"
}